{
  "gene_name": "Crossover junction endonuclease EME1",
  "term_label": "Holliday junction resolvase complex",
  "gene_symbol": "EME1",
  "term_id": "GO:0048476",
  "gene": "UniProtKB:Q96AY2"
}